{
  "term_id": "UNKNOWN:0002",
  "gene_symbol": "CENPL",
  "gene": "UniProtKB:Q8N0S6",
  "gene_name": "Centromere protein L",
  "term_label": "Unknown biological process"
}